{
  "term_label": "cytoplasm",
  "gene_name": "Protein Tob2",
  "term_id": "GO:0005737",
  "gene_symbol": "TOB2",
  "gene": "UniProtKB:Q14106"
}